inward rectifier potassium channel inhibitor activity [GO:0070320] (molecular function) Relationships: is a type of potassium channel inhibitor activity [GO:0019870]; negatively regulates GO:0005242 Definition: Binds to and stops, prevents, or reduces the activity of an inwardly rectifying potassium channel. Sources: GOC:mah